negative regulation of initiation of premeiotic DNA replication [GO:1904513] (biological process) Also known as: down regulation of initiation of premeiotic DNA replication, down regulation of premeiotic DNA replication initiation, down-regulation of initiation of premeiotic DNA replication, down-regulation of premeiotic DNA replication initiation, downregulation of initiation of premeiotic DNA replication, downregulation of premeiotic DNA replication initiation, negative regulation of premeiotic DNA replication initiation, inhibition of initiation of premeiotic DNA replication, inhibition of premeiotic DNA replication initiation, down regulation of initiation of meiotic DNA synthesis, down regulation of initiation of premeiotic DNA synthesis, down regulation of meiotic DNA replication initiation, down-regulation of initiation of meiotic DNA synthesis, down-regulation of initiation of premeiotic DNA synthesis, down-regulation of meiotic DNA replication initiation, downregulation of initiation of meiotic DNA synthesis, downregulation of initiation of premeiotic DNA synthesis, downregulation of meiotic DNA replication initiation, inhibition of initiation of meiotic DNA synthesis, inhibition of initiation of premeiotic DNA synthesis, inhibition of meiotic DNA replication initiation, negative regulation of initiation of meiotic DNA synthesis, negative regulation of initiation of premeiotic DNA synthesis, negative regulation of meiotic DNA replication initiation Definition: Any process that stops, prevents or reduces the frequency, rate or extent of initiation of premeiotic DNA replication. References: PMID:25891897 Sources: GOC:TermGenie, GO_REF:0000058 Relationships: is_a negative regulation of DNA-templated DNA replication initiation [GO:0032297]; is a type of negative regulation of meiotic cell cycle [GO:0051447]; is a type of negative regulation of nuclear cell cycle DNA replication [GO:1902576]; is a type of regulation of initiation of premeiotic DNA replication [GO:1904512]; RO_0002212 meiotic DNA replication initiation [GO:1902974]